{
  "term_id": "GO:0007417",
  "gene_symbol": "HTT",
  "gene_name": "Huntingtin",
  "term_label": "central nervous system development",
  "gene": "UniProtKB:P42858"
}